{
  "term_label": "telomere maintenance",
  "gene_symbol": "ATM",
  "gene_name": "Serine-protein kinase ATM",
  "term_id": "GO:0000723",
  "gene": "UniProtKB:Q13315"
}